{
  "term_id": "GO:0016529",
  "gene": "UniProtKB:Q8WXH0",
  "term_label": "sarcoplasmic reticulum",
  "gene_symbol": "SYNE2",
  "gene_name": "Nesprin-2"
}